DNA modification [GO:0006304] (biological process) Sources: GOC:jl, GOC:ma Relationships: is a type of DNA metabolic process [GO:0006259]; is a type of GO:0043412 Definition: The covalent alteration of one or more nucleotide sites in DNA, resulting in a change in its properties. Subtypes: DNA restriction-modification system [GO:0009307], DNA ADP-ribosylation [GO:0030592], DNA dealkylation [GO:0035510], DNA deamination [GO:0045006], depurination [GO:0045007], depyrimidination [GO:0045008], GO:0070580